negative regulation of bone mineralization [GO:0030502] (BP) Sources: GOC:go_curators Subtypes: negative regulation of bone mineralization involved in bone maturation [GO:1900158] Also known as: down regulation of bone mineralization, down-regulation of bone mineralization, downregulation of bone mineralization, inhibition of bone mineralization Relationships: is a type of GO:0030279; is a type of GO:0030500; is a type of GO:0070168; negatively regulates bone mineralization [GO:0030282] Definition: Any process that stops, prevents, or reduces the frequency, rate or extent of bone mineralization.